dTDP-4-amino-4,6-dideoxy-D-glucose transaminase activity [GO:0019179] (molecular function) Also known as: dTDP-4-amino-4,6-dideoxy-D-glucose aminotransferase activity, TDP-4-keto-6-deoxy-D-glucose transaminase activity, TDP-4-oxo-6-deoxy-D-glucose transaminase activity, dTDP-4-amino-4,6-dideoxy-D-glucose:2-oxoglutarate aminotransferase activity, thymidine diphospho-4-amino-4,6-dideoxyglucose aminotransferase activity, thymidine diphospho-4-amino-6-deoxyglucose aminotransferase activity, thymidine diphospho-4-keto-6-deoxy-D-glucose transaminase activity, thymidine diphospho-4-keto-6-deoxy-D-glucose-glutamic transaminase activity Relationships: is a type of GO:0008483 Definition: Catalysis of the reaction: dTDP-4-amino-4,6-dideoxy-D-glucose + 2-oxoglutarate = dTDP-4-dehydro-6-deoxy-D-glucose + L-glutamate. Sources: EC:2.6.1.33